metanephric extraglomerular mesangial cell proliferation involved in metanephros development [GO:0072261] (biological process) Also known as: metanephric Goormaghtigh proliferation, metanephric lacis cell proliferation Relationships: is a type of extraglomerular mesangial cell proliferation [GO:0072122]; is_a cell proliferation involved in metanephros development [GO:0072203]; is part of metanephric nephron development [GO:0072210] Sources: GOC:mtg_kidney_jan10 Definition: The multiplication or reproduction of extraglomerular glomerular mesangium cells in the metanephros by cell division, resulting in the expansion of their population. Extraglomerular mesangial cells (also known as lacis cells, Goormaghtigh cells) are light-staining cells in the kidney found outside the glomerulus, near the vascular pole and macula densa.